{
  "gene_symbol": "ANKLE2",
  "gene": "UniProtKB:Q86XL3",
  "term_id": "GO:0051721",
  "gene_name": "Ankyrin repeat and LEM domain-containing protein 2",
  "term_label": "protein phosphatase 2A binding"
}